postsynaptic density organization [GO:0097106] (biological process) Relationships: is a type of postsynaptic specialization organization [GO:0099084] Also known as: PSD organization, post synaptic density organization, post-synaptic density organization, postsynaptic density organisation References: PMID:21525273 Sources: GOC:BHF, GOC:sjp Subtypes: postsynaptic density assembly [GO:0097107], GO:0098880 Definition: A process that results in the assembly, arrangement of constituent parts, or disassembly of a postsynaptic density, a region that lies adjacent to the cytoplasmic face of the postsynaptic membrane at excitatory synapse. Regulation: regulated by regulation of postsynaptic density organization [GO:1905874]; negatively regulated by negative regulation of postsynaptic density organization [GO:1905875]; positively regulated by positive regulation of postsynaptic density organization [GO:1905876]